{
  "term_id": "GO:2000660",
  "gene_symbol": "OTUD4",
  "gene_name": "OTU domain-containing protein 4",
  "term_label": "negative regulation of interleukin-1-mediated signaling pathway",
  "gene": "UniProtKB:Q01804"
}